{
  "gene_symbol": "RGPD8",
  "gene_name": "RANBP2-like and GRIP domain-containing protein 8",
  "term_id": "GO:0006607",
  "gene": "UniProtKB:O14715",
  "term_label": "NLS-bearing protein import into nucleus"
}